{
  "gene": "UniProtKB:P01242",
  "term_label": "animal organ development",
  "gene_name": "Growth hormone variant",
  "term_id": "GO:0048513",
  "gene_symbol": "GH2"
}